myo-inositol hexakisphosphate biosynthetic process, via inositol 1,3,4-trisphosphate [GO:0033546] (biological process) Sources: GOC:mah, MetaCyc:PWY-6554 Definition: The chemical reactions and pathways resulting in the formation of 1D-myo-inositol 1,2,3,4,5,6-hexakisphosphate, phytate, by a pathway using inositol 1,4,5-trisphosphate produced from phosphatidylinositol 4,5-biphosphate hydrolysis by phospholipase C; in this pathway, inositol 1,4,5-trisphosphate is first converted to inositol 1,3,4-trisphosphate, and then phosphorylated further. Relationships: is_a GO:0033545 Also known as: myo-inositol hexakisphosphate anabolism, via inositol 1,3,4-trisphosphate, myo-inositol hexakisphosphate biosynthesis, via inositol 1,3,4-trisphosphate, myo-inositol hexakisphosphate formation, via inositol 1,3,4-trisphosphate, myo-inositol hexakisphosphate synthesis, via inositol 1,3,4-trisphosphate, phytate biosynthesis, via inositol 1,3,4-trisphosphate, phytate biosynthetic process, via inositol 1,3,4-trisphosphate